{
  "gene_symbol": "Q9Y3F1",
  "term_label": "Unknown molecular function",
  "gene_name": "Putative TAP2-associated 6.5 kDa polypeptide",
  "term_id": "UNKNOWN:0001",
  "gene": "UniProtKB:Q9Y3F1"
}